{
  "gene": "UniProtKB:Q8TCB7",
  "gene_name": "tRNA N(3)-methylcytidine methyltransferase METTL6",
  "gene_symbol": "METTL6",
  "term_id": "UNKNOWN:0002",
  "term_label": "Unknown biological process"
}